{
  "gene": "UniProtKB:Q9H3W5",
  "term_label": "Unknown biological process",
  "gene_symbol": "LRRN3",
  "gene_name": "Leucine-rich repeat neuronal protein 3",
  "term_id": "UNKNOWN:0002"
}